{
  "term_id": "UNKNOWN:0001",
  "term_label": "Unknown molecular function",
  "gene_symbol": "MGARP",
  "gene_name": "Protein MGARP",
  "gene": "UniProtKB:Q8TDB4"
}